{
  "gene_name": "Sodium channel protein type 11 subunit alpha",
  "term_id": "GO:0001518",
  "gene": "UniProtKB:Q9UI33",
  "gene_symbol": "SCN11A",
  "term_label": "voltage-gated sodium channel complex"
}